{
  "gene": "UniProtKB:Q8N743",
  "term_id": "GO:0005886",
  "gene_name": "Killer cell immunoglobulin-like receptor 3DL3",
  "gene_symbol": "KIR3DL3",
  "term_label": "plasma membrane"
}